{
  "gene_symbol": "TEX54",
  "gene": "UniProtKB:A0A1B0GVG6",
  "term_label": "Unknown biological process",
  "gene_name": "Testis-expressed protein 54",
  "term_id": "UNKNOWN:0002"
}